{
  "term_label": "RNA polymerase II transcription regulatory region sequence-specific DNA binding",
  "gene": "UniProtKB:A8K8V0",
  "term_id": "GO:0000977",
  "gene_name": "Zinc finger protein 785",
  "gene_symbol": "ZNF785"
}